{
  "term_id": "GO:0045087",
  "term_label": "innate immune response",
  "gene_name": "Immunity-related GTPase family M protein",
  "gene": "UniProtKB:A1A4Y4",
  "gene_symbol": "IRGM"
}